RNA biosynthetic process [GO:0032774] (biological process) Definition: The chemical reactions and pathways resulting in the formation of RNA, ribonucleic acid, one of the two main type of nucleic acid, consisting of a long, unbranched macromolecule formed from ribonucleotides joined in 3',5'-phosphodiester linkage. Includes polymerization of ribonucleotide monomers. Refers not only to transcription but also to e.g. viral RNA replication. Sources: GOC:mah, GOC:txnOH Also known as: RNA anabolism, RNA biosynthesis, RNA formation, RNA synthesis, double-stranded RNA biosynthesis, double-stranded RNA biosynthetic process, dsRNA biosynthesis, dsRNA biosynthetic process Note: Note that, in some cases, viral RNA replication and viral transcription from RNA actually refer to the same process, but may be called differently depending on the focus of a specific research study. Relationships: is a type of RNA metabolic process [GO:0016070]; is_a nucleic acid biosynthetic process [GO:0141187] Subtypes: promoter clearance during DNA-templated transcription [GO:0001109], RNA-templated transcription [GO:0001172], DNA-templated transcriptional start site selection [GO:0001173], maintenance of transcriptional fidelity during transcription elongation [GO:0001192], DNA replication, synthesis of primer [GO:0006269], DNA-templated transcription [GO:0006351], DNA-templated transcription initiation [GO:0006352], DNA-templated transcription termination [GO:0006353], DNA-templated transcription elongation [GO:0006354], viral RNA genome replication [GO:0039694], transcription pausing by RNA polymerase II [GO:0160239] Regulation: negatively regulated by negative regulation of RNA biosynthetic process [GO:1902679]; RO_0002213 by GO:1902680; regulated by regulation of RNA biosynthetic process [GO:2001141]